regulation of transcription elongation by RNA polymerase I [GO:2001207] (biological process) Subtypes: negative regulation of transcription elongation by RNA polymerase I [GO:2001208], positive regulation of transcription elongation by RNA polymerase I [GO:2001209] Relationships: is a type of regulation of DNA-templated transcription elongation [GO:0032784]; RO_0002211 transcription elongation by RNA polymerase I [GO:0006362] Also known as: regulation of RNA elongation from Pol I promoter, regulation of transcription elongation from RNA polymerase I promoter References: PMID:20299458 Definition: Any process that modulates the frequency, rate or extent of transcription elongation from RNA polymerase I promoter.